bile acid signaling pathway [GO:0038183] (biological process) References: PMID:12016314, PMID:36409000 Sources: GOC:signaling Relationships: is a type of signal transduction [GO:0007165] Note: This term is not for direct annotation. Please use a more specific child: 'cell surface bile acid receptor signaling pathway' for GPCRs and 'intracellular bile acid receptor signaling pathway' for nuclear receptors. Subtypes: adenylate cyclase-activating G protein-coupled bile acid receptor signaling pathway [GO:0038184], GO:0038185 Definition: The series of molecular signals initiated by bile acid binding to its receptor, and ending with the regulation of a downstream cellular process, e.g. transcription.